{
  "term_label": "regulation of transcription by RNA polymerase II",
  "term_id": "GO:0006357",
  "gene": "UniProtKB:Q8NI51",
  "gene_symbol": "CTCFL",
  "gene_name": "Transcriptional repressor CTCFL"
}